{
  "gene": "UniProtKB:Q9HCH3",
  "gene_symbol": "CPNE5",
  "term_label": "calcium-dependent phospholipid binding",
  "term_id": "GO:0005544",
  "gene_name": "Copine-5"
}